{
  "gene_name": "Follistatin",
  "term_id": "GO:0005615",
  "gene_symbol": "FST",
  "gene": "UniProtKB:P19883",
  "term_label": "extracellular space"
}